immune complex formation [GO:0097281] (biological process) Relationships: is a type of immunoglobulin mediated immune response [GO:0016064]; has part antigen binding [GO:0003823] Also known as: antibody-mediated agglutination Definition: The process that gives rise to an immune complex. Immune complexes are clusters of antibodies bound to antigen, to which complement may also be fixed, and which may precipitate or remain in solution. Examples are the clumping of cells such as bacteria or red blood cells in the presence of an antibody, precipitation of a toxin after an antibody binds to it, and clumping of viral particles as a result of antibody binding to the virus. Sources: GOC:add, GOC:rv